{
  "term_label": "Unknown cellular component",
  "gene_symbol": "ZNF861P",
  "gene": "UniProtKB:O60384",
  "term_id": "UNKNOWN:0003",
  "gene_name": "Putative zinc finger protein 861"
}